vanillin dehydrogenase activity [GO:0050608] (molecular function) Also known as: vanillin:NAD+ oxidoreductase activity Definition: Catalysis of the reaction: H2O + NAD+ + vanillin = 2 H+ + NADH + vanillate. Relationships: is a type of oxidoreductase activity, acting on the aldehyde or oxo group of donors, NAD or NADP as acceptor [GO:0016620] Sources: EC:1.2.1.67, RHEA:13309